{
  "term_label": "photoreceptor outer segment",
  "gene_symbol": "OPN1MW",
  "gene": "UniProtKB:P04001",
  "term_id": "GO:0001750",
  "gene_name": "Medium-wave-sensitive opsin 1"
}